lipoxin B4 metabolic process [GO:2001304] (biological process) Also known as: LXB4 metabolic process, LXB4 metabolism, lipoxin B4 metabolism Sources: GOC:mw Definition: The chemical reactions and pathways involving lipoxin B4. Lipoxin B4 is a C20 hydroxy fatty acid having (5S)-, (14R)- and (15S)-hydroxy groups as well as (6E)- (8Z)-, (10E)- and (12E)-double bonds. Relationships: is a type of long-chain fatty acid metabolic process [GO:0001676]; is_a GO:0033559; is_a fatty acid derivative metabolic process [GO:1901568] Subtypes: GO:2001306